{
  "term_id": "GO:0045585",
  "term_label": "positive regulation of cytotoxic T cell differentiation",
  "gene_symbol": "TNFSF9",
  "gene": "UniProtKB:P41273",
  "gene_name": "Tumor necrosis factor ligand superfamily member 9"
}